negative regulation of interleukin-8 production [GO:0032717] (biological process) Sources: GOC:mah Also known as: down regulation of interleukin-8 production, down-regulation of interleukin-8 production, downregulation of interleukin-8 production, negative regulation of IL-8 production, inhibition of interleukin-8 production, negative regulation of interleukin-8 biosynthetic process, negative regulation of interleukin-8 secretion Definition: Any process that stops, prevents, or reduces the frequency, rate, or extent of interleukin-8 production. Relationships: is a type of negative regulation of cytokine production [GO:0001818]; is_a regulation of interleukin-8 production [GO:0032677]; negatively regulates interleukin-8 production [GO:0032637]